{
  "term_id": "GO:0002312",
  "gene_symbol": "IFNA7",
  "gene_name": "Interferon alpha-7",
  "gene": "UniProtKB:P01567",
  "term_label": "B cell activation involved in immune response"
}